{
  "gene_symbol": "LINC00158",
  "term_label": "Unknown molecular function",
  "term_id": "UNKNOWN:0001",
  "gene": "UniProtKB:P58513",
  "gene_name": "Putative uncharacterized protein encoded by LINC00158"
}